{
  "term_label": "actin filament organization",
  "term_id": "GO:0007015",
  "gene_symbol": "TPM3",
  "gene": "UniProtKB:P06753",
  "gene_name": "Tropomyosin alpha-3 chain"
}